regulation of aggrephagy [GO:1905335] (BP) References: PMID:25686248 Sources: GOC:PARL, GOC:TermGenie, GOC:pad, GO_REF:0000058 Definition: Any process that modulates the frequency, rate or extent of aggrephagy. Relationships: is a type of regulation of macroautophagy [GO:0016241]; RO_0002211 aggrephagy [GO:0035973] Subtypes: negative regulation of aggrephagy [GO:1905336], GO:1905337